{
  "gene_symbol": "Q8N2B8",
  "gene_name": "Putative uncharacterized protein FLJ33534",
  "term_id": "UNKNOWN:0002",
  "term_label": "Unknown biological process",
  "gene": "UniProtKB:Q8N2B8"
}